leukotriene biosynthetic process [GO:0019370] (biological process) Definition: The chemical reactions and pathways resulting in the formation of leukotriene, a pharmacologically active substance derived from a polyunsaturated fatty acid, such as arachidonic acid. Relationships: is a type of GO:0006691; is a type of icosanoid biosynthetic process [GO:0046456] Subtypes: leukotriene B4 biosynthetic process [GO:0097251], leukotriene D4 biosynthetic process [GO:1901750], leukotriene A4 biosynthetic process [GO:1901753] Also known as: leukotriene anabolism, leukotriene biosynthesis, leukotriene formation, leukotriene synthesis Sources: GOC:go_curators